negative regulation of cell proliferation involved in kidney development [GO:1901723] (biological process) Subtypes: negative regulation of glomerular mesangial cell proliferation [GO:0072125], GO:2000607 References: PMID:18182616 Sources: GOC:TermGenie Also known as: down regulation of cell proliferation involved in kidney development, down-regulation of cell proliferation involved in kidney development, downregulation of cell proliferation involved in kidney development, inhibition of cell proliferation involved in kidney development Definition: Any process that stops, prevents or reduces the frequency, rate or extent of cell proliferation involved in kidney development. Relationships: is a type of GO:0008285; is a type of regulation of cell proliferation involved in kidney development [GO:1901722]; negatively regulates cell proliferation involved in kidney development [GO:0072111]